defense response to protozoan [GO:0042832] (biological process) Definition: Reactions triggered in response to the presence of a protozoan that act to protect the cell or organism. Sources: GOC:jl Relationships: is a type of response to protozoan [GO:0001562]; is a type of GO:0098542 Also known as: defence response to pathogenic protozoa, defence response to protozoa, defence response to protozoon, defense response to pathogenic protozoa, defense response to protozoa, defense response to protozoon, defense response to protozoan, incompatible interaction, resistance response to pathogenic protozoa, resistance response to pathogenic protozoan